secondary alcohol biosynthetic process [GO:1902653] (biological process) Definition: The chemical reactions and pathways resulting in the formation of secondary alcohol. Subtypes: cholesterol biosynthetic process [GO:0006695], ergosterol biosynthetic process [GO:0006696], ecdysone biosynthetic process [GO:0006697], menthol biosynthetic process [GO:0031525], butanediol biosynthetic process [GO:0034079], zymosterol biosynthetic process [GO:0036197], acetoin biosynthetic process [GO:0045151], 2-hydroxy-but-3-enyl glucosinolate biosynthetic process [GO:0080035], vomitoxin biosynthetic process [GO:0106110], culmorin biosynthetic process [GO:0106210], GO:0140872, conidiogenone biosynthetic process [GO:0140879], GO:1900554, GO:1900581, GO:1901755, propan-2-ol biosynthetic process [GO:1902640] Also known as: secondary alcohol anabolism, secondary alcohol biosynthesis, secondary alcohol formation, secondary alcohol synthesis References: PMID:11288200 Sources: GOC:TermGenie, GOC:mengo_curators, GO_REF:0000068 Relationships: is a type of alcohol biosynthetic process [GO:0046165]; is a type of secondary alcohol metabolic process [GO:1902652]